regulation of meiotic DNA double-strand break formation involved in reciprocal meiotic recombination [GO:1905261] (biological process) Subtypes: GO:0062209, negative regulation of meiotic DNA double-strand break formation involved in reciprocal meiotic recombination [GO:1905262], positive regulation of meiotic DNA double-strand break formation involved in reciprocal meiotic recombination [GO:1905263] Relationships: is a type of regulation of meiotic DNA double-strand break formation [GO:1903341]; is part of reciprocal meiotic recombination [GO:0007131]; regulates meiotic DNA double-strand break formation involved in reciprocal meiotic recombination [GO:0010780] Definition: Any process that modulates the frequency, rate or extent of meiotic DNA double-strand break formation involved in reciprocal meiotic recombination. References: PMID:26653857 Sources: GOC:TermGenie, GO_REF:0000058